interleukin-19 receptor binding [GO:0045516] (molecular function) Relationships: is_a cytokine receptor binding [GO:0005126] Sources: GOC:go_curators Also known as: IL-19, interleukin-19 receptor ligand Definition: Binding to an interleukin-19 receptor.